{
  "gene_symbol": "ARHGAP26",
  "term_id": "UNKNOWN:0003",
  "gene": "UniProtKB:Q9UNA1",
  "term_label": "Unknown cellular component",
  "gene_name": "Rho GTPase-activating protein 26"
}